collagen type VII trimer [GO:0005590] (cellular component) References: PMID:19693541 Definition: A collagen homotrimer of alpha1(VII) chains; type VII collagen triple helices form antiparallel dimer, which in turn associate laterally to form anchoring fibrils that connect type IV collagen in the basal lamina to plaques in the underlying connective tissue. It binds laminin. Relationships: is a type of GO:0140158; is part of collagen type VII anchoring fibril [GO:0098652]